histone H3K9 demethylase activity [GO:0032454] (molecular function) Relationships: is a type of histone H3 demethylase activity [GO:0141052] References: PMID:16362057 Note: Comment: Note that the residue position corresponds to the canonical human H3 histone (UniProtKB:P84243); this residue is conserved across all eukaryotes. Residue 1 is the first residue following removal of the initiating Methionine (Met). Note that each histone is encoded by multiple genes, and sequences may vary across different genes within an organism. Also known as: histone H3-K49 demethylase activity, histone H3-methyl-lysine-9 demethylase activity, histone demethylase activity (H3-K9 specific) Subtypes: histone H3K9me/H3K9me2 demethylase activity [GO:0140683], histone H3K9me2/H3K9me3 demethylase activity [GO:0140684], FAD-dependent histone H3K9me/H3K9me2 demethylase activity [GO:0140685] Definition: Catalysis of the removal of a methyl group from a modified lysine residue at position 9 of the histone H3 protein.